{
  "gene_name": "Steryl-sulfatase",
  "gene": "UniProtKB:P08842",
  "gene_symbol": "STS",
  "term_id": "GO:0004065",
  "term_label": "arylsulfatase activity"
}